{
  "gene": "UniProtKB:Q9H0A0",
  "term_label": "rRNA acetylation involved in maturation of SSU-rRNA",
  "gene_symbol": "NAT10",
  "gene_name": "RNA cytidine acetyltransferase",
  "term_id": "GO:1904812"
}